{
  "term_id": "GO:0006357",
  "term_label": "regulation of transcription by RNA polymerase II",
  "gene_symbol": "ZNF587",
  "gene_name": "Zinc finger protein 587",
  "gene": "UniProtKB:Q96SQ5"
}